{
  "term_id": "UNKNOWN:0002",
  "gene": "UniProtKB:Q8IYM0",
  "term_label": "Unknown biological process",
  "gene_name": "Protein FAM186B",
  "gene_symbol": "FAM186B"
}